{
  "gene": "UniProtKB:P05538",
  "gene_name": "HLA class II histocompatibility antigen, DQ beta 2 chain",
  "gene_symbol": "HLA-DQB2",
  "term_id": "GO:0023026",
  "term_label": "MHC class II protein complex binding"
}